{
  "gene_name": "Keratin-associated protein 19-8",
  "term_id": "UNKNOWN:0001",
  "gene_symbol": "KRTAP19-8",
  "gene": "UniProtKB:Q3LI54",
  "term_label": "Unknown molecular function"
}